{
  "gene": "UniProtKB:O76075",
  "term_id": "GO:0006309",
  "gene_symbol": "DFFB",
  "gene_name": "DNA fragmentation factor subunit beta",
  "term_label": "apoptotic DNA fragmentation"
}